chromosome passenger complex localization to kinetochore [GO:0072356] (biological process) Definition: A cellular protein complex localization that acts on a chromosome passenger complex; as a result, the complex is transported to, or maintained in, a specific location at the kinetochore. A chromosome passenger complex is a protein complex that contains the BIR-domain-containing protein Survivin, Aurora B kinase, INCENP and Borealin, and coordinates various events based on its location to different structures during the course of mitosis. Also known as: CPC complex localization to kinetochore, CPC localization to kinetochore, chromosomal passenger complex localization to kinetochore, chromosome passenger complex localisation to kinetochore Sources: GOC:mah Regulation: positively regulated by GO:0140430 Relationships: is a type of protein-containing complex localization [GO:0031503]; is a type of protein localization to kinetochore [GO:0034501]